{
  "gene": "UniProtKB:O43448",
  "term_label": "potassium channel regulator activity",
  "gene_name": "Voltage-gated potassium channel subunit beta-3",
  "gene_symbol": "KCNAB3",
  "term_id": "GO:0015459"
}